{
  "gene_name": "Exportin-T",
  "term_label": "tRNA binding",
  "gene": "UniProtKB:O43592",
  "term_id": "GO:0000049",
  "gene_symbol": "XPOT"
}